{
  "gene_symbol": "PRPF6",
  "gene": "UniProtKB:O94906",
  "term_label": "mRNA splicing, via spliceosome",
  "term_id": "GO:0000398",
  "gene_name": "Pre-mRNA-processing factor 6"
}